3'-5' DNA helicase activity [GO:0043138] (molecular function) Relationships: is a type of DNA helicase activity [GO:0003678] Sources: EC:5.6.2.4, GOC:jl Also known as: 3' to 5' DNA helicase activity, ATP-dependent 3' to 5' DNA helicase activity, ATP-dependent 3'-5' DNA helicase activity Definition: Unwinding a DNA helix in the direction 5' to 3', driven by ATP hydrolysis. Subtypes: single-stranded 3'-5' DNA helicase activity [GO:1990518]